{
  "gene_name": "Tetratricopeptide repeat protein 14",
  "term_id": "UNKNOWN:0002",
  "gene": "UniProtKB:Q96N46",
  "term_label": "Unknown biological process",
  "gene_symbol": "TTC14"
}